glucan 1,4-alpha-maltohexaosidase activity [GO:0033927] (molecular function) Relationships: is_a hydrolase activity, hydrolyzing O-glycosyl compounds [GO:0004553] Sources: EC:3.2.1.98 Also known as: 1,4-alpha-D-glucan maltohexaohydrolase activity, G6-amylase activity, exo-maltohexaohydrolase activity, maltohexaose-producing amylase activity Definition: Catalysis of the hydrolysis of (1->4)-alpha-D-glucosidic linkages in amylaceous polysaccharides, to remove successive maltohexaose residues from the non-reducing chain ends.